negative regulation of D-glucose transmembrane transport [GO:0010829] (biological process) Definition: Any process that decreases the frequency, rate or extent of glucose transport across a membrane. Glucose transport is the directed movement of the hexose monosaccharide glucose into, out of or within a cell, or between cells, by means of some agent such as a transporter or pore. Sources: GOC:BHF, GOC:dph, GOC:tb Also known as: negative regulation of glucose transmembrane transport, negative regulation of glucose transport Relationships: is a type of GO:0010827; is a type of GO:0034763; negatively regulates D-glucose transmembrane transport [GO:1904659] Subtypes: negative regulation of D-glucose import [GO:0046325]